positive regulation of voltage-gated sodium channel activity [GO:1905152] (biological process) Also known as: positive regulation of voltage gated sodium channel activity, positive regulation of voltage-dependent sodium channel activity, positive regulation of voltage-gated sodium ion channel activity, positive regulation of voltage-sensitive sodium channel, up regulation of voltage gated sodium channel activity, up regulation of voltage-dependent sodium channel activity, up regulation of voltage-gated sodium channel activity, up regulation of voltage-gated sodium ion channel activity, up regulation of voltage-sensitive sodium channel, up-regulation of voltage gated sodium channel activity, up-regulation of voltage-dependent sodium channel activity, up-regulation of voltage-gated sodium channel activity, up-regulation of voltage-gated sodium ion channel activity, up-regulation of voltage-sensitive sodium channel, upregulation of voltage gated sodium channel activity, upregulation of voltage-dependent sodium channel activity, upregulation of voltage-gated sodium channel activity, upregulation of voltage-gated sodium ion channel activity, upregulation of voltage-sensitive sodium channel, activation of voltage gated sodium channel activity, activation of voltage-dependent sodium channel activity, activation of voltage-gated sodium channel activity, activation of voltage-gated sodium ion channel activity, activation of voltage-sensitive sodium channel Definition: Any process that activates or increases the frequency, rate or extent of voltage-gated sodium channel activity. References: PMID:24198377 Sources: GOC:TermGenie, GO_REF:0000059 Relationships: is a type of regulation of voltage-gated sodium channel activity [GO:1905150]; is a type of GO:2000651; is a type of positive regulation of cation channel activity [GO:2001259]; positively regulates voltage-gated sodium channel activity [GO:0005248]